regulation of stress response to copper ion [GO:1903853] (biological process) References: PMID:23437011 Sources: GOC:TermGenie, GOC:kmv, GO_REF:0000058 Subtypes: negative regulation of stress response to copper ion [GO:1903854], positive regulation of stress response to copper ion [GO:1903855] Definition: Any process that modulates the frequency, rate or extent of stress response to copper ion. Also known as: regulation of stress response to copper, regulation of response to copper ion stress, regulation of response to copper toxicity Relationships: is a type of GO:0080134; regulates stress response to copper ion [GO:1990169]